{
  "gene": "UniProtKB:A6NCI8",
  "gene_name": "Uncharacterized protein C2orf78",
  "term_label": "Unknown cellular component",
  "gene_symbol": "C2orf78",
  "term_id": "UNKNOWN:0003"
}